regulation of olfactory learning [GO:0090328] (biological process) Sources: GOC:dph, GOC:tb Definition: Any process that modulates the rate, frequency, or extent of olfactory learning. Olfactory learning is any process in an organism in which a relatively long-lasting adaptive behavioral change occurs in response to (repeated) exposure to an olfactory cue. Relationships: is a type of regulation of nervous system process [GO:0031644]; is a type of regulation of response to stimulus [GO:0048583]; is a type of regulation of behavior [GO:0050795]; regulates olfactory learning [GO:0008355]